type III interferon binding [GO:0034347] (molecular function) Relationships: is a type of interferon binding [GO:0019961] Also known as: interferon-lambda binding Note: Note that IL-28A, IL-28B, and IL-29 are types of interferon-lambda. References: PMID:15546383, PMID:16734557 Sources: GOC:add, ISBN:0126896631 Definition: Binding to a type III interferon. Interferon lambda is the only member of the type III interferon found so far.